meiotic chromosome segregation [GO:0045132] (biological process) Subtypes: male meiosis chromosome segregation [GO:0007060], female meiosis chromosome segregation [GO:0016321], GO:0032837, homologous chromosome segregation [GO:0045143], meiotic sister chromatid segregation [GO:0045144] Sources: GOC:ai, GOC:mah Definition: The process in which genetic material, in the form of chromosomes, is organized into specific structures and then physically separated and apportioned to two or more sets during M phase of the meiotic cell cycle. Relationships: is a type of nuclear chromosome segregation [GO:0098813]; is a type of meiotic cell cycle process [GO:1903046]; is part of meiotic nuclear division [GO:0140013]